{
  "term_label": "Unknown biological process",
  "term_id": "UNKNOWN:0002",
  "gene_symbol": "MTMR12",
  "gene": "UniProtKB:Q9C0I1",
  "gene_name": "Myotubularin-related protein 12"
}